cellular response to interleukin-13 [GO:0035963] (biological process) References: PMID:20100461 Sources: GOC:sjw Relationships: is a type of response to interleukin-13 [GO:0035962]; is a type of cellular response to cytokine stimulus [GO:0071345] Also known as: cellular response to IL-13 Definition: Any process that results in a change in state or activity of a cell (in terms of movement, secretion, enzyme production, gene expression, etc.) as a result of an interleukin-13 stimulus.